{
  "term_label": "Unknown molecular function",
  "term_id": "UNKNOWN:0001",
  "gene_name": "Disrupted in renal carcinoma protein 1",
  "gene_symbol": "DIRC1",
  "gene": "UniProtKB:Q969H9"
}